maintenance of animal organ identity [GO:0048496] (biological process) Sources: GOC:tb Definition: The process in which the identity of an animal organ is maintained. Identity is considered to be the aggregate of characteristics by which a structure is recognized. Subtypes: maintenance of kidney identity [GO:0072005] Relationships: is a type of GO:0045596; is part of GO:0048513